5,6,7,8-tetrahydrosarcinapterin catabolic process [GO:1901854] (biological process) Relationships: is a type of GO:0006796; is a type of GO:0042560; is a type of organophosphate catabolic process [GO:0046434]; is a type of GO:0072352 Definition: The chemical reactions and pathways resulting in the breakdown of 5,6,7,8-tetrahydrosarcinapterin. Also known as: 5,6,7,8-tetrahydrosarcinapterin breakdown, 5,6,7,8-tetrahydrosarcinapterin catabolism, 5,6,7,8-tetrahydrosarcinapterin degradation Sources: GOC:TermGenie, GOC:yaf, UniPathway:UPA00069